{
  "gene_name": "Variable charge X-linked protein 2",
  "term_label": "Unknown cellular component",
  "gene_symbol": "VCX2",
  "term_id": "UNKNOWN:0003",
  "gene": "UniProtKB:Q9H322"
}